{
  "gene": "UniProtKB:P05546",
  "term_id": "GO:0005615",
  "gene_name": "Heparin cofactor 2",
  "term_label": "extracellular space",
  "gene_symbol": "SERPIND1"
}